{
  "gene": "UniProtKB:Q7Z442",
  "term_id": "GO:0005262",
  "gene_name": "Polycystin-1-like protein 2",
  "gene_symbol": "PKD1L2",
  "term_label": "calcium channel activity"
}